{
  "term_label": "ADP-ribose diphosphatase activity",
  "term_id": "GO:0047631",
  "gene": "UniProtKB:P53370",
  "gene_name": "Nucleoside diphosphate-linked moiety X motif 6",
  "gene_symbol": "NUDT6"
}